{
  "gene_name": "Cholesterol 25-hydroxylase",
  "term_label": "C-4 methylsterol oxidase activity",
  "term_id": "GO:0000254",
  "gene_symbol": "CH25H",
  "gene": "UniProtKB:O95992"
}